{
  "gene_name": "Arginine--tRNA ligase, cytoplasmic",
  "term_label": "arginine-tRNA ligase activity",
  "gene": "UniProtKB:P54136",
  "term_id": "GO:0004814",
  "gene_symbol": "RARS1"
}